positive regulation of voltage-gated chloride channel activity [GO:1902943] (biological process) References: PMID:22006324 Sources: GOC:TermGenie, GOC:als, GO_REF:0000059 Relationships: is a type of GO:1901529; positively regulates GO:0005247 Definition: Any process that activates or increases the frequency, rate or extent of voltage-gated chloride channel activity. Also known as: positive regulation of voltage gated chloride channel activity, positive regulation of voltage-dependent chloride channel activity, up regulation of voltage gated chloride channel activity, up regulation of voltage-dependent chloride channel activity, up regulation of voltage-gated chloride channel activity, up-regulation of voltage gated chloride channel activity, up-regulation of voltage-dependent chloride channel activity, up-regulation of voltage-gated chloride channel activity, upregulation of voltage gated chloride channel activity, upregulation of voltage-dependent chloride channel activity, upregulation of voltage-gated chloride channel activity, activation of voltage gated chloride channel activity, activation of voltage-dependent chloride channel activity, activation of voltage-gated chloride channel activity